{
  "term_id": "GO:0000981",
  "gene_name": "Cyclic AMP-dependent transcription factor ATF-6 alpha",
  "gene": "UniProtKB:P18850",
  "gene_symbol": "ATF6",
  "term_label": "DNA-binding transcription factor activity, RNA polymerase II-specific"
}